establishment or maintenance of monopolar cell polarity [GO:0061339] (biological process) Subtypes: establishment of monopolar cell polarity [GO:0061162], establishment or maintenance of monopolar cell polarity regulating cell shape [GO:0061340] Relationships: is a type of GO:0007163 Definition: Any cellular process that results in the specification, formation or maintenance of monopolar intracellular organization or cell growth patterns. Monopolar cell organization is directional organization along an axis. Sources: GOC:dph, GOC:vw